{
  "term_id": "GO:0005544",
  "gene_name": "Synaptotagmin-8",
  "term_label": "calcium-dependent phospholipid binding",
  "gene": "UniProtKB:Q8NBV8",
  "gene_symbol": "SYT8"
}